{
  "gene_name": "Carbohydrate sulfotransferase 1",
  "term_label": "Unknown cellular component",
  "gene": "UniProtKB:O43916",
  "gene_symbol": "CHST1",
  "term_id": "UNKNOWN:0003"
}